negative regulation of circadian sleep/wake cycle, sleep [GO:0042321] (biological process) Definition: Any process that stops, prevents or reduces the duration or quality of sleep, a readily reversible state of reduced awareness and metabolic activity that occurs periodically in many animals. Also known as: down regulation of circadian sleep/wake cycle, sleep, down-regulation of circadian sleep/wake cycle, sleep, downregulation of circadian sleep/wake cycle, sleep, negative regulation of sleep, inhibition of circadian sleep/wake cycle, sleep Relationships: is a type of negative regulation of circadian rhythm [GO:0042754]; is_a regulation of circadian sleep/wake cycle, sleep [GO:0045187]; is a type of negative regulation of behavior [GO:0048521]; negatively regulates circadian sleep/wake cycle, sleep [GO:0050802] Sources: GOC:go_curators, GOC:jl, ISBN:0192800981 Subtypes: negative regulation of circadian sleep/wake cycle, REM sleep [GO:0042322], negative regulation of circadian sleep/wake cycle, non-REM sleep [GO:0042323]